{
  "term_label": "norepinephrine binding",
  "term_id": "GO:0051380",
  "gene": "UniProtKB:P07550",
  "gene_name": "Beta-2 adrenergic receptor",
  "gene_symbol": "ADRB2"
}